DUBm complex [GO:0071819] (cellular component) Definition: A protein complex that forms part of SAGA-type complexes SAGA and SLIK, and mediates deubiquitination of histone H2B. In S. cerevisiae, the DUBm consists of the proteins Ubp8p, Sgf11p, Sus1p, and Sgf73p. References: PMID:19226466, PMID:20395473 Also known as: deubiquitinating module, deubiquitination module, SAGA DUBm complex Relationships: is a type of nuclear protein-containing complex [GO:0140513]